{
  "gene_name": "Cullin-2",
  "term_id": "GO:0005634",
  "gene_symbol": "CUL2",
  "term_label": "nucleus",
  "gene": "UniProtKB:Q13617"
}